{
  "gene": "UniProtKB:P02461",
  "term_id": "GO:0030020",
  "term_label": "extracellular matrix structural constituent conferring tensile strength",
  "gene_symbol": "COL3A1",
  "gene_name": "Collagen alpha-1(III) chain"
}